{
  "gene_name": "Putative DBH-like monooxygenase protein 2",
  "gene": "UniProtKB:A6NHM9",
  "term_id": "GO:0005507",
  "gene_symbol": "MOXD2P",
  "term_label": "copper ion binding"
}